organelle lumen [GO:0043233] (cellular component) Sources: GOC:jl, GOC:mah Relationships: is_a membrane-enclosed lumen [GO:0031974]; is part of organelle [GO:0043226] Definition: The internal volume enclosed by the membranes of a particular organelle; includes the volume enclosed by a single organelle membrane, e.g. endoplasmic reticulum lumen, or the volume enclosed by the innermost of the two lipid bilayers of an organelle envelope, e.g. nuclear lumen. Subtypes: GO:0031983, rhoptry lumen [GO:0034591], intracellular organelle lumen [GO:0070013], GO:0120203